{
  "gene": "UniProtKB:Q9NX09",
  "term_id": "UNKNOWN:0003",
  "gene_name": "DNA damage-inducible transcript 4 protein",
  "gene_symbol": "DDIT4",
  "term_label": "Unknown cellular component"
}